{
  "term_label": "binding of sperm to zona pellucida",
  "gene": "UniProtKB:P60852",
  "term_id": "GO:0007339",
  "gene_name": "Zona pellucida sperm-binding protein 1",
  "gene_symbol": "ZP1"
}